rolling hairpin viral DNA replication [GO:0039685] (biological process) Definition: A viral DNA replication process where a 3' hairpin structure in the viral single-stranded DNA (ssDNA) template serves as a primer for host enzymes to synthesize DNA. Also known as: ssDNA rolling hairpin viral DNA replication Relationships: is a type of viral DNA genome replication [GO:0039693] Sources: GOC:bf, GOC:jl, VZ:2656